crotonyl-CoA reductase activity [GO:0043880] (molecular function) Also known as: CCR, crotonyl-coenzyme A reductase activity Definition: Catalysis of the reaction: butanoyl-CoA + NADP+ = (2E)-butenoyl-CoA + NADPH + H+. (2E)-butenoyl-CoA is also called crotonyl-CoA. Relationships: is a type of GO:0016628 References: PMID:11162231 Sources: RHEA:27906